{
  "gene_name": "DENN domain-containing protein 1A",
  "term_label": "cytosol",
  "gene": "UniProtKB:Q8TEH3",
  "term_id": "GO:0005829",
  "gene_symbol": "DENND1A"
}